{
  "gene_name": "Glutamate receptor ionotropic, NMDA 3B",
  "term_id": "GO:0098839",
  "gene_symbol": "GRIN3B",
  "term_label": "postsynaptic density membrane",
  "gene": "UniProtKB:O60391"
}